{
  "gene": "UniProtKB:Q9BXL8",
  "gene_name": "Cell division cycle-associated protein 4",
  "term_label": "cytoplasm",
  "gene_symbol": "CDCA4",
  "term_id": "GO:0005737"
}